{
  "term_id": "GO:0019731",
  "gene_name": "Elafin",
  "gene": "UniProtKB:P19957",
  "gene_symbol": "PI3",
  "term_label": "antibacterial humoral response"
}